{
  "term_label": "nervous system development",
  "gene": "UniProtKB:Q9H8V3",
  "term_id": "GO:0007399",
  "gene_symbol": "ECT2",
  "gene_name": "Protein ECT2"
}